{
  "gene_symbol": "RAB5B",
  "gene": "UniProtKB:P61020",
  "gene_name": "Ras-related protein Rab-5B",
  "term_label": "GTPase activity",
  "term_id": "GO:0003924"
}